protein localization to condensed chromosome [GO:1903083] (biological process) Subtypes: protein localization to kinetochore [GO:0034501], GO:1903084 Relationships: is a type of protein localization to chromosome [GO:0034502] Definition: A process in which a protein is transported to, or maintained in, a location within a condensed chromosome. Also known as: protein localisation in condensed chromosome, protein localisation to condensed chromosome, protein localization in condensed chromosome References: PMID:12707312 Sources: GOC:TermGenie, GOC:kmv, GO_REF:0000087